N-ethylammeline chlorohydrolase activity [GO:0016217] (molecular function) Relationships: is_a hydrolase activity, acting on acid halide bonds, in C-halide compounds [GO:0019120] Sources: MetaCyc:R465-RXN Definition: Catalysis of the reaction: deethylsimazine + H2O = N-ethylammeline + chloride + H+.